{
  "gene_symbol": "HIGD1B",
  "term_id": "GO:0005739",
  "gene_name": "HIG1 domain family member 1B",
  "gene": "UniProtKB:Q9P298",
  "term_label": "mitochondrion"
}